{
  "gene_name": "Zinc finger HIT domain-containing protein 1",
  "gene": "UniProtKB:O43257",
  "gene_symbol": "ZNHIT1",
  "term_label": "nucleosome binding",
  "term_id": "GO:0031491"
}